raffinose-raffinose alpha-galactotransferase activity [GO:0047234] (molecular function) Definition: Catalysis of the reaction: 2 raffinose = sucrose + 1F-alpha-D-galactosylraffinose. Also known as: raffinose-raffinose a-galactosyltransferase activity, raffinose-raffinose alpha-galactosyltransferase activity, raffinose (raffinose donor) galactosyltransferase activity, raffinose:raffinose alpha-D-galactosyltransferase activity, raffinose:raffinose alpha-galactosyltransferase activity Relationships: is_a galactosyltransferase activity [GO:0008378] Sources: EC:2.4.1.166